{
  "term_label": "Unknown cellular component",
  "term_id": "UNKNOWN:0003",
  "gene_symbol": "TMEM169",
  "gene_name": "Transmembrane protein 169",
  "gene": "UniProtKB:Q96HH4"
}